{
  "term_id": "UNKNOWN:0001",
  "gene_symbol": "C16orf86",
  "gene": "UniProtKB:Q6ZW13",
  "gene_name": "Uncharacterized protein C16orf86",
  "term_label": "Unknown molecular function"
}